ergosteryl 3-beta-D-glucoside biosynthetic process [GO:1904463] (biological process) Also known as: ergosteryl 3-beta-D-glucoside anabolism, ergosteryl 3-beta-D-glucoside biosynthesis, ergosteryl 3-beta-D-glucoside formation, ergosteryl 3-beta-D-glucoside synthesis Definition: The chemical reactions and pathways resulting in the formation of ergosteryl 3-beta-D-glucoside. References: PMID:26116408 Sources: GOC:TermGenie, GO_REF:0000068 Relationships: is a type of GO:0006694; is a type of saponin biosynthetic process [GO:0016135]; is a type of beta-glucoside biosynthetic process [GO:1901806]